{
  "term_label": "Unknown cellular component",
  "gene_symbol": "DNAJC5G",
  "gene_name": "DnaJ homolog subfamily C member 5G",
  "gene": "UniProtKB:Q8N7S2",
  "term_id": "UNKNOWN:0003"
}